{
  "term_label": "intracellular signal transduction",
  "gene_symbol": "STK10",
  "gene_name": "Serine_threonine-protein kinase 10",
  "gene": "UniProtKB:O94804",
  "term_id": "GO:0035556"
}